{
  "gene": "UniProtKB:P18074",
  "term_id": "GO:0005634",
  "term_label": "nucleus",
  "gene_symbol": "ERCC2",
  "gene_name": "General transcription and DNA repair factor IIH helicase subunit XPD"
}